{
  "gene_symbol": "BSDC1",
  "term_label": "Unknown biological process",
  "gene_name": "BSD domain-containing protein 1",
  "gene": "UniProtKB:Q9NW68",
  "term_id": "UNKNOWN:0002"
}